{
  "term_id": "GO:0030837",
  "gene": "UniProtKB:Q76I76",
  "gene_symbol": "SSH2",
  "term_label": "negative regulation of actin filament polymerization",
  "gene_name": "Protein phosphatase Slingshot homolog 2"
}